regulation of epithelial cell proliferation [GO:0050678] (biological process) Sources: GOC:ai Definition: Any process that modulates the frequency, rate or extent of epithelial cell proliferation. Relationships: is a type of GO:0042127; regulates epithelial cell proliferation [GO:0050673] Subtypes: regulation of endothelial cell proliferation [GO:0001936], regulation of keratinocyte proliferation [GO:0010837], regulation of mammary gland epithelial cell proliferation [GO:0033599], regulation of urothelial cell proliferation [GO:0050675], GO:0050679, negative regulation of epithelial cell proliferation [GO:0050680], regulation of epithelial cell proliferation involved in prostate gland development [GO:0060768], regulation of type B pancreatic cell proliferation [GO:0061469], regulation of synoviocyte proliferation [GO:1901645], GO:1904002, regulation of cholangiocyte proliferation [GO:1904054], regulation of granulosa cell proliferation [GO:1904195], GO:1904441, regulation of acinar cell proliferation [GO:1904697], regulation of hepatocyte proliferation [GO:2000345], regulation of epithelial cell proliferation involved in lung morphogenesis [GO:2000794], regulation of lens epithelial cell proliferation [GO:2001109]